{
  "term_id": "GO:0160184",
  "gene": "UniProtKB:P56746",
  "gene_symbol": "CLDN15",
  "gene_name": "Claudin-15",
  "term_label": "paracellular transport"
}